{
  "gene": "UniProtKB:Q03923",
  "gene_symbol": "ZNF85",
  "term_label": "RNA polymerase II cis-regulatory region sequence-specific DNA binding",
  "term_id": "GO:0000978",
  "gene_name": "Zinc finger protein 85"
}